{
  "term_id": "GO:1904714",
  "gene_symbol": "GFAP",
  "term_label": "regulation of chaperone-mediated autophagy",
  "gene_name": "Glial fibrillary acidic protein",
  "gene": "UniProtKB:P14136"
}